N,N'-diacetylbacillosaminyl-diphospho-undecaprenol alpha-1,3-N-acetylgalactosaminyltransferase activity [GO:0102335] (molecular function) Definition: Catalysis of the reaction: N,N'-diacetyl-alpha-D-bacillosaminyl-diphospho-tri-trans,hepta-cis-undecaprenol + UDP-N-acetyl-D-galactosamine = N-acetyl-D-galactosaminyl-alpha-(1->3)-N,N'-diacetyl-alpha-D-bacillosaminyl-diphospho-tri-trans,hepta-cis-undecaprenol + UDP + H+. Relationships: is a type of hexosyltransferase activity [GO:0016758] Sources: EC:2.4.1.290, GOC:pz